cellular response to tellurium ion [GO:0071293] (biological process) Sources: GOC:mah Definition: Any process that results in a change in state or activity of a cell (in terms of movement, secretion, enzyme production, gene expression, etc.) as a result of a tellurium ion stimulus. Also known as: cellular response to tellurium Relationships: is a type of response to tellurium ion [GO:0046690]; is a type of cellular response to metal ion [GO:0071248]; is a type of cellular response to oxygen-containing compound [GO:1901701]